neuron projection maintenance [GO:1990535] (biological process) Definition: The organization process that preserves a neuron projection in a stable functional or structural state. A neuron projection is a prolongation or process extending from a nerve cell, e.g. an axon or dendrite. Relationships: is a type of neuron projection organization [GO:0106027] References: PMID:25359212 Sources: GOC:kmv Also known as: neuron process maintenance, neuron protrusion maintenance, neuronal cell projection maintenance, neurite maintenance, axon homeostasis, axon maintenance